{
  "gene_name": "Cytochrome P450 26B1",
  "gene": "UniProtKB:Q9NR63",
  "term_label": "retinoic acid catabolic process",
  "term_id": "GO:0034653",
  "gene_symbol": "CYP26B1"
}